{
  "term_label": "cytosolic large ribosomal subunit",
  "gene_symbol": "RPL18A",
  "gene": "UniProtKB:Q02543",
  "term_id": "GO:0022625",
  "gene_name": "Large ribosomal subunit protein eL20"
}